{
  "gene_symbol": "NAGPA",
  "gene_name": "N-acetylglucosamine-1-phosphodiester alpha-N-acetylglucosaminidase",
  "term_label": "secretion of lysosomal enzymes",
  "term_id": "GO:0033299",
  "gene": "UniProtKB:Q9UK23"
}